{
  "gene_symbol": "GP9",
  "term_id": "UNKNOWN:0002",
  "term_label": "Unknown biological process",
  "gene": "UniProtKB:P14770",
  "gene_name": "Platelet glycoprotein IX"
}